xanthine phosphoribosyltransferase activity [GO:0000310] (molecular function) Relationships: is a type of purine phosphoribosyltransferase activity [GO:0106130] Also known as: xanthine-guanine phosphoribosyltransferase activity, 5-phospho-alpha-D-ribose-1-diphosphate:xanthine phospho-D-ribosyltransferase activity, XMP pyrophosphorylase activity, XMP:diphosphate 5-phospho-alpha-D-ribosyltransferase activity, Xan phosphoribosyltransferase activity, xanthosine 5'-phosphate pyrophosphorylase activity, xanthylate pyrophosphorylase activity, xanthylic pyrophosphorylase activity Sources: RHEA:10800 Definition: Catalysis of the reaction: diphosphate + XMP = 5-phospho-alpha-D-ribose 1-diphosphate + xanthine.